{
  "gene": "UniProtKB:Q9UHC6",
  "gene_symbol": "CNTNAP2",
  "term_id": "UNKNOWN:0001",
  "gene_name": "Contactin-associated protein-like 2",
  "term_label": "Unknown molecular function"
}